{
  "term_label": "Unknown biological process",
  "term_id": "UNKNOWN:0002",
  "gene_name": "Olfactory receptor 6C74",
  "gene_symbol": "OR6C74",
  "gene": "UniProtKB:A6NCV1"
}